{
  "term_label": "Unknown molecular function",
  "gene_symbol": "ICOS",
  "term_id": "UNKNOWN:0001",
  "gene": "UniProtKB:Q9Y6W8",
  "gene_name": "Inducible T-cell costimulator"
}